{
  "term_id": "UNKNOWN:0003",
  "gene_name": "Putative uncharacterized protein encoded by LINC00482",
  "gene_symbol": "LINC00482",
  "term_label": "Unknown cellular component",
  "gene": "UniProtKB:Q8N8I6"
}